organic acid:sodium symporter activity [GO:0005343] (molecular function) Also known as: sodium:dicarboxylate/tricarboxylate symporter activity, sodium/chloride-dependent organic acid cotransporter activity Sources: TC:2.A.28.1.1 Definition: Enables the transfer of a solute or solutes from one side of a membrane to the other according to the reaction: organic acid(out) + Na+(out) = organic acid(in) + Na+(in). Subtypes: proline:sodium symporter activity [GO:0005298], creatine:sodium symporter activity [GO:0005309], GO:0005369, L-ascorbate:sodium symporter activity [GO:0008520], glycine:sodium symporter activity [GO:0015375], GO:0015498, glutamate:sodium symporter activity [GO:0015501], alanine:sodium symporter activity [GO:0015655], branched-chain amino acid:sodium symporter activity [GO:0015657], sodium:dicarboxylate symporter activity [GO:0017153], monocarboxylate:sodium symporter activity [GO:0140161] Relationships: is a type of GO:0015370